5-aminolevulinate synthase activity [GO:0003870] (molecular function) Definition: Catalysis of the reaction: glycine + H+ + succinyl-CoA = 5-aminolevulinate + CO2 + CoA. Relationships: is a type of N-succinyltransferase activity [GO:0016749] Also known as: 5-aminolevulinate synthetase activity, 5-aminolevulinic acid synthase activity, 5-aminolevulinic acid synthetase activity, ALA synthase activity, ALA synthetase activity, ALAS activity, alpha-aminolevulinic acid synthase activity, aminolevulinate synthase activity, aminolevulinate synthetase activity, aminolevulinic acid synthase activity, aminolevulinic acid synthetase activity, aminolevulinic synthetase activity, delta-ALA synthetase activity, delta-aminolevulinate synthase activity, delta-aminolevulinate synthetase activity, delta-aminolevulinic acid synthase activity, delta-aminolevulinic acid synthetase activity, delta-aminolevulinic synthetase activity, succinyl-CoA:glycine C-succinyltransferase (decarboxylating) Sources: EC:2.3.1.37, RHEA:12921